{
  "gene_name": "Growth_differentiation factor 15",
  "gene_symbol": "GDF15",
  "term_id": "GO:0005615",
  "gene": "UniProtKB:Q99988",
  "term_label": "extracellular space"
}